{
  "gene": "UniProtKB:P12544",
  "gene_symbol": "GZMA",
  "term_id": "GO:0140507",
  "term_label": "granzyme-mediated programmed cell death signaling pathway",
  "gene_name": "Granzyme A"
}